callose deposition in cell wall [GO:0052543] (biological process) Subtypes: defense response by callose deposition in cell wall [GO:0052544] Also known as: callose localization in cell wall, cell wall callose deposition, cell wall callose localization Relationships: is a type of cell wall thickening [GO:0052386]; is a type of callose localization [GO:0052545] Sources: GOC:mtg_pamgo_17jul06 Definition: Any process in which callose is transported to, and/or maintained in, the cell wall. Callose is a linear 1,3-beta-d-glucan formed from UDP-glucose and is found in certain plant cell walls.